{
  "gene_symbol": "KCNK10",
  "gene": "UniProtKB:P57789",
  "term_label": "outward rectifier potassium channel activity",
  "gene_name": "Potassium channel subfamily K member 10",
  "term_id": "GO:0015271"
}